{
  "gene": "UniProtKB:Q8IX21",
  "gene_name": "SMC5-SMC6 complex localization factor protein 2",
  "term_id": "UNKNOWN:0001",
  "gene_symbol": "SLF2",
  "term_label": "Unknown molecular function"
}